{
  "gene_name": "Olfactory receptor 52W1",
  "term_id": "GO:0004984",
  "gene_symbol": "OR52W1",
  "gene": "UniProtKB:Q6IF63",
  "term_label": "olfactory receptor activity"
}